{
  "gene_symbol": "PLCL2",
  "term_id": "GO:0032228",
  "gene_name": "Inactive phospholipase C-like protein 2",
  "term_label": "regulation of synaptic transmission, GABAergic",
  "gene": "UniProtKB:Q9UPR0"
}